{
  "gene": "UniProtKB:P49257",
  "term_label": "Golgi membrane",
  "gene_symbol": "LMAN1",
  "term_id": "GO:0000139",
  "gene_name": "Protein ERGIC-53"
}